{
  "term_label": "protein serine/threonine phosphatase activity",
  "gene": "UniProtKB:Q15750",
  "gene_symbol": "TAB1",
  "term_id": "GO:0004722",
  "gene_name": "TGF-beta-activated kinase 1 and MAP3K7-binding protein 1"
}